{
  "gene_name": "Pre-mRNA-processing factor 39",
  "term_id": "GO:0000395",
  "gene_symbol": "PRPF39",
  "term_label": "mRNA 5'-splice site recognition",
  "gene": "UniProtKB:Q86UA1"
}